{
  "gene_name": "Protein FAM13C",
  "gene": "UniProtKB:Q8NE31",
  "term_label": "Unknown biological process",
  "term_id": "UNKNOWN:0002",
  "gene_symbol": "FAM13C"
}